{
  "gene_name": "Glutathione S-transferase theta-2B",
  "term_label": "glutathione metabolic process",
  "term_id": "GO:0006749",
  "gene_symbol": "GSTT2B",
  "gene": "UniProtKB:P0CG30"
}